{
  "gene": "UniProtKB:Q6UX34",
  "term_id": "UNKNOWN:0002",
  "gene_name": "Protein SNORC",
  "term_label": "Unknown biological process",
  "gene_symbol": "SNORC"
}